{
  "gene_symbol": "SARNP",
  "gene": "UniProtKB:P82979",
  "term_id": "UNKNOWN:0001",
  "gene_name": "SAP domain-containing ribonucleoprotein",
  "term_label": "Unknown molecular function"
}